peptide pheromone receptor activity [GO:0036318] (molecular function) Relationships: is a type of GO:0008528; is_a pheromone receptor activity [GO:0016503] Subtypes: mating-type a-factor pheromone receptor activity [GO:0004933], mating-type alpha-factor pheromone receptor activity [GO:0004934], mating-type M-factor pheromone receptor activity [GO:0036319], GO:0036320 Sources: GOC:al Definition: Combining with a peptide pheromone, and transmitting the signal across the membrane to initiate a change in cell activity.